{
  "term_id": "GO:1990756",
  "gene_name": "DET1 homolog",
  "gene_symbol": "DET1",
  "gene": "UniProtKB:Q7L5Y6",
  "term_label": "ubiquitin-like ligase-substrate adaptor activity"
}